{
  "term_label": "cell adhesion molecule binding",
  "gene_name": "Teneurin-4",
  "gene_symbol": "TENM4",
  "gene": "UniProtKB:Q6N022",
  "term_id": "GO:0050839"
}